{
  "gene_name": "Mediator of RNA polymerase II transcription subunit 1",
  "term_label": "nuclear thyroid hormone receptor binding",
  "gene": "UniProtKB:Q15648",
  "term_id": "GO:0046966",
  "gene_symbol": "MED1"
}